{
  "term_label": "extracellular space",
  "gene_symbol": "HP",
  "term_id": "GO:0005615",
  "gene": "UniProtKB:P00738",
  "gene_name": "Haptoglobin"
}